dorsal motor nucleus of vagus nerve morphogenesis [GO:0035762] (biological process) Sources: GOC:dgh Definition: The process in which the dorsal motor nucleus of the vagus nerve is generated and organized. Morphogenesis pertains to the creation of form. Relationships: is a type of anatomical structure morphogenesis [GO:0009653]; is part of dorsal motor nucleus of vagus nerve development [GO:0021744]